{
  "gene_symbol": "TFAP2A",
  "gene_name": "Transcription factor AP-2-alpha",
  "term_label": "nervous system development",
  "term_id": "GO:0007399",
  "gene": "UniProtKB:P05549"
}